{
  "term_id": "GO:0001228",
  "gene_name": "Basic helix-loop-helix domain-containing protein USF3",
  "gene_symbol": "USF3",
  "gene": "UniProtKB:Q68DE3",
  "term_label": "DNA-binding transcription activator activity, RNA polymerase II-specific"
}